{
  "gene_symbol": "DNAJC5",
  "term_label": "presynapse",
  "term_id": "GO:0098793",
  "gene_name": "DnaJ homolog subfamily C member 5",
  "gene": "UniProtKB:Q9H3Z4"
}